{
  "gene_symbol": "AVPR1A",
  "gene_name": "Vasopressin V1a receptor",
  "term_label": "G protein-coupled receptor signaling pathway",
  "gene": "UniProtKB:P37288",
  "term_id": "GO:0007186"
}